{
  "term_id": "GO:0005737",
  "gene_symbol": "MARCHF8",
  "gene": "UniProtKB:Q5T0T0",
  "term_label": "cytoplasm",
  "gene_name": "E3 ubiquitin-protein ligase MARCHF8"
}